1,4-dihydroxy-2-naphthoyl-CoA thioesterase activity [GO:0061522] (molecular function) Definition: Catalysis of the reaction 1,4-dihydroxy-2-naphthoyl-CoA + H2O = 1,4-dihydroxy-2-naphthoate + CoA + H+. Sources: RHEA:26309 Relationships: is a type of acyl-CoA hydrolase activity [GO:0016289]